{
  "term_label": "RNA export from nucleus",
  "term_id": "GO:0006405",
  "gene_symbol": "NUP98",
  "gene": "UniProtKB:P52948",
  "gene_name": "Nuclear pore complex protein Nup98-Nup96"
}